aminomethyltransferase activity [GO:0004047] (molecular function) Relationships: is a type of hydroxymethyl-, formyl- and related transferase activity [GO:0016742] Also known as: S-aminomethyldihydrolipoylprotein:(6S)-tetrahydrofolate aminomethyltransferase (ammonia-forming) activity, T-protein, glycine synthase activity, glycine-cleavage system T-protein activity, protein-8-S-aminomethyldihydrolipoyllysine:tetrahydrofolate aminomethyltransferase (ammonia-forming) activity, protein-S8-aminomethyldihydrolipoyllysine:tetrahydrofolate aminomethyltransferase (ammonia-forming) activity, tetrahydrofolate aminomethyltransferase activity Definition: Catalysis of the reaction: N(6)-[(R)-S(8)-aminomethyldihydrolipoyl]-L-lysyl-[protein] + (6S)-5,6,7,8-tetrahydrofolate = N(6)-[(R)-dihydrolipoyl]-L-lysyl-[protein] + (6R)-5,10-methylene-5,6,7,8-tetrahydrofolate + NH4+. Sources: RHEA:16945